dihydrofolate synthase activity [GO:0008841] (MF) Also known as: 7,8-dihydrofolate synthetase activity, 7,8-dihydropteroate:L-glutamate ligase (ADP) activity, 7,8-dihydropteroate:L-glutamate ligase (ADP-forming), DHFS activity, FHFS activity, FHFS/FPGS activity, H(2)-folate synthetase activity, H2-folate synthetase activity, dihydrofolate synthetase activity, dihydrofolate synthetase-folylpolyglutamate synthetase activity, dihydropteroate:L-glutamate ligase (ADP-forming) activity, folylpoly-(gamma-glutamate) synthetase-dihydrofolate synthase activity Relationships: is a type of GO:0016881; is part of GO:0006761 Sources: EC:6.3.2.12 Definition: Catalysis of the reaction: ATP + dihydropterate + L-glutamate = ADP + phosphate + dihydrofolate.